swim bladder morphogenesis [GO:0048795] (biological process) Sources: GOC:mh Definition: The process in which the anatomical structure of the swim bladder is generated and organized. The swim bladder is used by some fishes to maintain buoyancy and may function in addition as a sound producing organ, a sound receptor, and a respiratory organ. Also known as: gas bladder morphogenesis Relationships: is_a animal organ morphogenesis [GO:0009887]; is part of swim bladder development [GO:0048794]